{
  "term_id": "GO:0005737",
  "gene_name": "Thioredoxin reductase 3",
  "gene_symbol": "TXNRD3",
  "term_label": "cytoplasm",
  "gene": "UniProtKB:Q86VQ6"
}